{
  "gene": "UniProtKB:P29762",
  "term_id": "GO:0001972",
  "gene_symbol": "CRABP1",
  "term_label": "retinoic acid binding",
  "gene_name": "Cellular retinoic acid-binding protein 1"
}